{
  "term_id": "UNKNOWN:0001",
  "gene_symbol": "OCSTAMP",
  "term_label": "Unknown molecular function",
  "gene_name": "Osteoclast stimulatory transmembrane protein",
  "gene": "UniProtKB:Q9BR26"
}